{
  "gene_symbol": "FKRP",
  "gene": "UniProtKB:Q9H9S5",
  "term_id": "GO:0000139",
  "term_label": "Golgi membrane",
  "gene_name": "Ribitol 5-phosphate transferase FKRP"
}